zinc ion transmembrane transporter activity [GO:0005385] (molecular function) Subtypes: high-affinity zinc transmembrane transporter activity [GO:0000006], low-affinity zinc ion transmembrane transporter activity [GO:0000007], GO:0015633, GO:0016463, zinc efflux transmembrane transporter activity [GO:0022883], zinc:bicarbonate symporter activity [GO:0140412], GO:0140826 Definition: Enables the transfer of zinc (Zn) ions from one side of a membrane to the other. Relationships: is a type of transition metal ion transmembrane transporter activity [GO:0046915]; is part of zinc ion transmembrane transport [GO:0071577] Sources: GOC:dgf Also known as: zinc, iron permease activity, cobalt, zinc uptake permease activity, zinc, cadmium uptake permease activity, zinc, cadmium, cobalt, nickel, lead-efflux ATPase activity